{
  "term_id": "UNKNOWN:0002",
  "term_label": "Unknown biological process",
  "gene": "UniProtKB:P02747",
  "gene_name": "Complement C1q subcomponent subunit C",
  "gene_symbol": "C1QC"
}